{
  "term_id": "UNKNOWN:0003",
  "gene": "UniProtKB:Q9UNU6",
  "gene_name": "7-alpha-hydroxycholest-4-en-3-one 12-alpha-hydroxylase",
  "gene_symbol": "CYP8B1",
  "term_label": "Unknown cellular component"
}